{
  "term_label": "methyl-CpG binding",
  "gene_name": "Putative methyl-CpG-binding domain protein 3-like 5",
  "gene": "UniProtKB:A6NJ08",
  "term_id": "GO:0008327",
  "gene_symbol": "MBD3L5"
}